{
  "term_label": "adenosine 5'-(hexahydrogen pentaphosphate) catabolic process",
  "gene": "UniProtKB:A0A024RBG1",
  "gene_symbol": "NUDT4B",
  "gene_name": "Diphosphoinositol polyphosphate phosphohydrolase NUDT4B",
  "term_id": "GO:1901911"
}